{
  "term_label": "nucleus",
  "gene_symbol": "CHML",
  "term_id": "GO:0005634",
  "gene_name": "Rab proteins geranylgeranyltransferase component A 2",
  "gene": "UniProtKB:P26374"
}